D-arabitol catabolic process to D-xylulose 5-phosphate [GO:0019528] (biological process) Relationships: is a type of GO:0051159; is a type of D-xylulose 5-phosphate metabolic process [GO:0051167] Definition: The chemical reactions and pathways resulting in the breakdown of D-arabitol to form D-xylulose 5-phosphate. D-arabitol is converted into D-xylulose, which is then phosphorylated to form D-xylulose-5-phosphate. Sources: MetaCyc:DARABITOLUTIL-PWY Also known as: D-arabitol breakdown to xylulose 5-phosphate, D-arabitol degradation to xylulose 5-phosphate, D-arabitol degradation, D-arabitol utilization